{
  "gene_name": "Kinetochore-associated protein 1",
  "gene_symbol": "KNTC1",
  "term_label": "cytoplasm",
  "term_id": "GO:0005737",
  "gene": "UniProtKB:P50748"
}